{
  "gene": "UniProtKB:Q16695",
  "gene_name": "Histone H3.1t",
  "gene_symbol": "H3-4",
  "term_label": "heterochromatin formation",
  "term_id": "GO:0031507"
}